{
  "gene_symbol": "ZNF662",
  "term_label": "RNA polymerase II cis-regulatory region sequence-specific DNA binding",
  "term_id": "GO:0000978",
  "gene": "UniProtKB:Q6ZS27",
  "gene_name": "Zinc finger protein 662"
}